{
  "gene_symbol": "TBC1D10A",
  "gene": "UniProtKB:Q9BXI6",
  "term_label": "GTPase activator activity",
  "term_id": "GO:0005096",
  "gene_name": "TBC1 domain family member 10A"
}